glycerol catabolic process [GO:0019563] (biological process) Subtypes: aerobic glycerol catabolic process [GO:0019564], anaerobic glycerol catabolic process [GO:0019588], glycolytic process from glycerol [GO:0061613] Definition: The chemical reactions and pathways resulting in the breakdown of glycerol, 1,2,3-propanetriol, a sweet, hygroscopic, viscous liquid, widely distributed in nature as a constituent of many lipids. Sources: GOC:go_curators, ISBN:0198506732 Also known as: glycerol breakdown, glycerol catabolism, glycerol degradation Relationships: is a type of GO:0006071; is a type of alditol catabolic process [GO:0019405]